{
  "gene_symbol": "TREX2",
  "gene": "UniProtKB:Q9BQ50",
  "term_id": "GO:0006308",
  "term_label": "DNA catabolic process",
  "gene_name": "Three prime repair exonuclease 2"
}